response to cAMP [GO:0051591] (biological process) Subtypes: GO:0031319, cellular response to cAMP [GO:0071320] Sources: GOC:ai Relationships: is a type of GO:0014074; is a type of response to organophosphorus [GO:0046683]; is a type of response to oxygen-containing compound [GO:1901700] Also known as: response to 3',5' cAMP, response to 3',5'-cAMP, response to adenosine 3',5'-cyclophosphate, response to cyclic AMP Definition: Any process that results in a change in state or activity of a cell or an organism (in terms of movement, secretion, enzyme production, gene expression, etc.) as a result of a cAMP (cyclic AMP, adenosine 3',5'-cyclophosphate) stimulus.